response to simvastatin [GO:1903491] (BP) Relationships: is a type of response to lipid [GO:0033993]; is a type of response to statin [GO:0036273] Note: Note that this term is in the subset of terms that should not be used for direct manual annotation of gene products. It was created to be used for cross-referencing by other ontologies. Direct annotations to this term may be amended during annotation QC. Definition: Any process that results in a change in state or activity of a cell or an organism (in terms of movement, secretion, enzyme production, gene expression, etc.) as a result of a simvastatin stimulus. Simvastatin is a statin used as a cholesterol-lowering and anti-cardiovascular disease drug. References: PMID:23100282 Sources: GOC:TermGenie, GOC:sl, GO_REF:0000071